{
  "term_id": "GO:0005634",
  "gene_symbol": "BCL11A",
  "gene_name": "B-cell lymphoma_leukemia 11A",
  "gene": "UniProtKB:Q9H165",
  "term_label": "nucleus"
}